{
  "term_label": "cell adhesion",
  "gene_name": "CCN family member 1",
  "term_id": "GO:0007155",
  "gene_symbol": "CCN1",
  "gene": "UniProtKB:O00622"
}